{
  "term_label": "guanyl-nucleotide exchange factor activity",
  "gene_symbol": "LOC107987545",
  "gene": "UniProtKB:A0A2R8YFR7",
  "term_id": "GO:0005085",
  "gene_name": "DH domain-containing protein"
}